tetrahydrobiopterin metabolic process [GO:0046146] (biological process) Subtypes: tetrahydrobiopterin biosynthetic process [GO:0006729], tetrahydrobiopterin catabolic process [GO:0046147] Relationships: is a type of diol metabolic process [GO:0034311]; is a type of GO:0042558 Also known as: 5,6,7,8-tetrahydrobiopterin metabolic process, tetrahydrobiopterin metabolism Definition: The chemical reactions and pathways involving tetrahydrobiopterin, the reduced form of biopterin (2-amino-4-hydroxy-6-(1,2-dihydroxypropyl)-pteridine). It functions as a hydroxylation coenzyme, e.g. in the conversion of phenylalanine to tyrosine. References: PMID:21871890